{
  "gene_symbol": "ALPK3",
  "gene": "UniProtKB:Q96L96",
  "term_id": "GO:0055013",
  "gene_name": "Alpha-protein kinase 3",
  "term_label": "cardiac muscle cell development"
}